{
  "term_label": "endopeptidase activity",
  "term_id": "GO:0004175",
  "gene_name": "Phosphoinositide-3-kinase-interacting protein 1",
  "gene_symbol": "PIK3IP1",
  "gene": "UniProtKB:Q96FE7"
}